{
  "term_id": "GO:0051028",
  "gene_name": "RNA-binding protein FXR2",
  "gene": "UniProtKB:P51116",
  "term_label": "mRNA transport",
  "gene_symbol": "FXR2"
}